{
  "gene_name": "Potassium voltage-gated channel subfamily A member 6",
  "term_label": "membrane",
  "term_id": "GO:0016020",
  "gene_symbol": "KCNA6",
  "gene": "UniProtKB:P17658"
}